{
  "gene_symbol": "ACP3",
  "term_label": "plasma membrane",
  "term_id": "GO:0005886",
  "gene": "UniProtKB:P15309",
  "gene_name": "Prostatic acid phosphatase"
}